lactosylceramide 4-alpha-galactosyltransferase activity [GO:0050512] (molecular function) Also known as: lactosylceramide 4-a-galactosyltransferase activity, globotriaosylceramide/CD77 synthase activity, histo-blood group P(k) UDP-galactose activity, Gal-beta-(1,4)-Glc-beta-1-Cer alpha-(1,4)-galactosyltransferase activity, Gal-beta-1,4-Glc-beta-1-Cer alpha-1,4-galactosyltransferase activity, UDP-galactose:lactosylceramide 4II-alpha-D-galactosyltransferase activity, histo-blood group Pk UDP-galactose Relationships: is a type of UDP-galactosyltransferase activity [GO:0035250] Definition: Catalysis of the reaction: beta-D-galactosyl-(1,4)-D-glucosylceramide + UDP-galactose = alpha-D-galactosyl-(1,4)-beta-D-galactosyl-(1,4)-D-glucosylceramide + UDP. Sources: EC:2.4.1.228, MetaCyc:2.4.1.228-RXN